{
  "gene_name": "Protein S100-A1",
  "term_label": "sarcoplasmic reticulum",
  "gene_symbol": "S100A1",
  "term_id": "GO:0016529",
  "gene": "UniProtKB:P23297"
}